{
  "gene_symbol": "PHF23",
  "gene_name": "PHD finger protein 23",
  "term_id": "GO:0031398",
  "term_label": "positive regulation of protein ubiquitination",
  "gene": "UniProtKB:Q9BUL5"
}